{
  "term_id": "GO:0005794",
  "gene_name": "Amyloid beta precursor like protein 1",
  "term_label": "Golgi apparatus",
  "gene_symbol": "APLP1",
  "gene": "UniProtKB:P51693"
}